{
  "term_id": "UNKNOWN:0003",
  "gene_symbol": "TRAJ42",
  "gene_name": "T cell receptor alpha joining 42",
  "term_label": "Unknown cellular component",
  "gene": "UniProtKB:A0A075B6Y9"
}